monoatomic ion homeostasis [GO:0050801] (BP) Sources: GOC:ai Definition: Any process involved in the maintenance of an internal steady state of monoatomic ions within an organism or cell. Monatomic ions (also called simple ions) are ions consisting of exactly one atom. Also known as: ion homeostasis, electrolyte homeostasis, negative regulation of crystal formation, regulation of ion homeostasis Relationships: is a type of GO:0048878 Subtypes: intracellular monoatomic ion homeostasis [GO:0006873], monoatomic cation homeostasis [GO:0055080], monoatomic anion homeostasis [GO:0055081]